{
  "gene_name": "AP2-associated protein kinase 1",
  "gene_symbol": "AAK1",
  "term_id": "GO:0035612",
  "term_label": "AP-2 adaptor complex binding",
  "gene": "UniProtKB:Q2M2I8"
}